{
  "term_id": "GO:0045103",
  "gene": "UniProtKB:Q9H7C4",
  "gene_name": "Syncoilin",
  "term_label": "intermediate filament-based process",
  "gene_symbol": "SYNC"
}